{
  "gene_symbol": "IGLV3-22",
  "term_label": "immunoglobulin complex",
  "gene": "UniProtKB:A0A075B6J6",
  "term_id": "GO:0019814",
  "gene_name": "Immunoglobulin lambda variable 3-22"
}